{
  "gene_symbol": "VSIG2",
  "term_label": "Unknown biological process",
  "term_id": "UNKNOWN:0002",
  "gene_name": "V-set and immunoglobulin domain-containing protein 2",
  "gene": "UniProtKB:Q96IQ7"
}